{
  "gene_symbol": "SMDT1",
  "gene_name": "Essential MCU regulator, mitochondrial",
  "gene": "UniProtKB:Q9H4I9",
  "term_id": "GO:0051560",
  "term_label": "mitochondrial calcium ion homeostasis"
}